{
  "gene_symbol": "SVOP",
  "term_id": "UNKNOWN:0001",
  "gene_name": "Synaptic vesicle 2-related protein",
  "gene": "UniProtKB:Q8N4V2",
  "term_label": "Unknown molecular function"
}